corticotropin hormone receptor binding [GO:0031780] (MF) Sources: GOC:dph, GOC:mah, GOC:nln Definition: Binding to a corticotropin hormone receptor. Also known as: ACTH receptor binding, adrenocorticotropin hormone receptor binding, adrenocorticotropin receptor binding, corticotropin receptor binding, adrenocorticotropic hormone receptor ligand Relationships: is a type of melanocortin receptor binding [GO:0031779]